supramolecular fiber organization [GO:0097435] (biological process) Regulation: regulated by regulation of supramolecular fiber organization [GO:1902903]; negatively regulated by negative regulation of supramolecular fiber organization [GO:1902904]; positively regulated by positive regulation of supramolecular fiber organization [GO:1902905] Definition: A process that is carried out at the cellular level which results in the assembly, arrangement of constituent parts, or disassembly of a supramolecular fiber, a polymer consisting of an indefinite number of protein or protein complex subunits that have polymerised to form a fiber-shaped structure. Sources: GOC:pr Also known as: extracellular fibril organisation, extracellular fibril organization, extracellular fibril organization and biogenesis, fibril organisation, fibril organization Relationships: is a type of cellular component organization [GO:0016043] Subtypes: actin filament organization [GO:0007015], microtubule depolymerization [GO:0007019], myofibril assembly [GO:0030239], myosin filament organization [GO:0031033], GO:0031122, intermediate filament organization [GO:0045109], GO:0046785, GO:0048251, cytoophidium organization [GO:0140904], microfibril assembly [GO:0160054], fibronectin fibril organization [GO:1905590], intranuclear rod assembly [GO:1905861], amyloid fibril formation [GO:1990000]